{
  "gene_name": "EH domain-containing protein 3",
  "gene_symbol": "EHD3",
  "term_label": "perinuclear region of cytoplasm",
  "term_id": "GO:0048471",
  "gene": "UniProtKB:Q9NZN3"
}